nucleoside oxidase activity [GO:0033715] (molecular function) Sources: EC:1.1.3.28, RHEA:28651 Definition: Catalysis of the reactions: inosine + O2 = 9-riburonosylhypoxanthine + 2 H2O; (1a) 2 inosine + O2 = 2 5'-dehydroinosine + 2 H2O, and (1b) 2 5'-dehydroinosine + O2 = 2 9-riburonosylhypoxanthine + 2 H2O. Relationships: is a type of oxidoreductase activity, acting on the CH-OH group of donors, oxygen as acceptor [GO:0016899] Also known as: nucleoside:oxygen 5'-oxidoreductase activity